positive regulation of bacterial-type flagellum assembly [GO:1902210] (biological process) Also known as: positive regulation of bacterial flagellum assembly, up regulation of bacterial flagellum assembly, up regulation of bacterial-type flagellum assembly, up-regulation of bacterial flagellum assembly, up-regulation of bacterial-type flagellum assembly, upregulation of bacterial flagellum assembly, upregulation of bacterial-type flagellum assembly, activation of bacterial flagellum assembly, activation of bacterial-type flagellum assembly Relationships: is a type of GO:0031346; is_a positive regulation of organelle assembly [GO:1902117]; is a type of regulation of bacterial-type flagellum assembly [GO:1902208]; RO_0002213 GO:0044780 Definition: Any process that activates or increases the frequency, rate or extent of bacterial-type flagellum assembly. Sources: GOC:TermGenie, GOC:jl